{
  "gene_symbol": "TIGAR",
  "term_label": "fructose-2,6-bisphosphate 2-phosphatase activity",
  "term_id": "GO:0004331",
  "gene": "UniProtKB:Q9NQ88",
  "gene_name": "Fructose-2,6-bisphosphatase TIGAR"
}